negative regulation of nematode pharynx morphogenesis [GO:0110042] (biological process) References: PMID:20805556 Sources: GOC:rz Definition: Any process that stops, prevents, or reduces the frequency, rate or extent of nematode pharynx morphogenesis. Relationships: is a type of regulation of nematode pharynx morphogenesis [GO:0110041]; is a type of negative regulation of animal organ morphogenesis [GO:0110111]; negatively regulates nematode pharynx morphogenesis [GO:0110040]